{
  "term_id": "GO:0005925",
  "gene_name": "Inactive tyrosine-protein kinase PEAK1",
  "term_label": "focal adhesion",
  "gene": "UniProtKB:Q9H792",
  "gene_symbol": "PEAK1"
}